{
  "gene": "UniProtKB:Q9BVC3",
  "term_label": "maintenance of mitotic sister chromatid cohesion",
  "gene_symbol": "DSCC1",
  "gene_name": "Sister chromatid cohesion protein DCC1",
  "term_id": "GO:0034088"
}